iron ion import across plasma membrane [GO:0098711] (BP) Regulation: regulated by regulation of iron ion import across plasma membrane [GO:1904438]; negatively regulated by negative regulation of iron ion import across plasma membrane [GO:1904439]; positively regulated by GO:1904440 Subtypes: heme import across plasma membrane [GO:1904334] References: PMID:8321236 Sources: GOC:mah Relationships: is a type of GO:0033212; is a type of GO:0034755; is a type of inorganic cation import across plasma membrane [GO:0098659] Also known as: iron ion import into cell, ferrous ion import into cell, ferrous iron import across plasma membrane, ferrous iron import into cell, iron import into cell Definition: The directed movement of iron ions from outside of a cell, across the plasma membrane and into the cytosol.